S-nitrosoglutathione reductase (NADPH) activity [GO:0160163] (molecular function) Relationships: is a type of GO:0016616 Definition: Catalysis of the reaction: H+ + NADPH + S-nitrosoglutathione = NADP+ + S-(hydroxysulfenamide)glutathione. Sources: RHEA:63500